{
  "gene_symbol": "NXF3",
  "term_label": "RNA binding",
  "term_id": "GO:0003723",
  "gene": "UniProtKB:Q9H4D5",
  "gene_name": "Nuclear RNA export factor 3"
}